{
  "gene_name": "IQ motif and SEC7 domain-containing protein 2",
  "term_label": "vesicle-mediated transport",
  "gene_symbol": "IQSEC2",
  "gene": "UniProtKB:Q5JU85",
  "term_id": "GO:0016192"
}